regulation of presynaptic active zone assembly [GO:1905518] (biological process) Definition: Any process that modulates the frequency, rate or extent of presynaptic active zone assembly. References: PMID:15797875 Sources: GOC:BHF, GOC:TermGenie, GOC:rl, GO_REF:0000058 Also known as: regulation of pre-synaptic active zone assembly, regulation of pre-synaptic active zone formation, regulation of presynaptic active zone formation, regulation of pre-synaptic active zone component assembly, regulation of pre-synaptic active zone component formation Relationships: is a type of regulation of cellular component organization [GO:0051128]; regulates presynaptic active zone assembly [GO:1904071] Subtypes: negative regulation of presynaptic active zone assembly [GO:1905519], GO:1905520